{
  "term_id": "GO:0048477",
  "gene_symbol": "NANOS1",
  "gene": "UniProtKB:Q8WY41",
  "term_label": "oogenesis",
  "gene_name": "Nanos homolog 1"
}